{
  "term_id": "GO:0035556",
  "term_label": "intracellular signal transduction",
  "gene_name": "Protein kinase C alpha type",
  "gene": "UniProtKB:P17252",
  "gene_symbol": "PRKCA"
}